{
  "gene": "UniProtKB:O94911",
  "gene_symbol": "ABCA8",
  "term_label": "ATPase-coupled transmembrane transporter activity",
  "gene_name": "ABC-type organic anion transporter ABCA8",
  "term_id": "GO:0042626"
}